{
  "gene_symbol": "DBT",
  "gene": "UniProtKB:P11182",
  "term_label": "mitochondrion",
  "gene_name": "Lipoamide acyltransferase component of branched-chain alpha-keto acid dehydrogenase complex, mitochondrial",
  "term_id": "GO:0005739"
}